formate transport [GO:0015724] (biological process) Sources: GOC:krc Subtypes: formic acid secretion [GO:0046721] Definition: The directed movement of formate into, out of or within a cell, or between cells, by means of some agent such as a transporter or pore. Relationships: is a type of monocarboxylic acid transport [GO:0015718]